dibenzothiophene monooxygenase activity [GO:0018640] (MF) Relationships: is a type of oxidoreductase activity, acting on paired donors, with incorporation or reduction of molecular oxygen, reduced flavin or flavoprotein as one donor, and incorporation of one atom of oxygen [GO:0016712] Definition: Catalysis of the reaction: dibenzothiophene + FMNH2 + O2 = dibenzothiophene 5-oxide + FMN + H2O + H+. Sources: RHEA:49076